high-affinity L-glutamate transmembrane transporter activity [GO:0005314] (molecular function) Sources: TC:2.A.3.10.5 Definition: Enables the transfer of glutamate from one side of a membrane to the other. In high-affinity transport the transporter is able to bind the solute even if it is only present at very low concentrations. Also known as: high-affinity glutamate transmembrane transporter activity, high-affinity glutamate transporter activity Relationships: is a type of L-glutamate transmembrane transporter activity [GO:0005313]; is a type of glutamate:sodium symporter activity [GO:0015501]